{
  "term_id": "GO:0033130",
  "term_label": "acetylcholine receptor binding",
  "gene_name": "Lymphocyte antigen 6 family member G6E",
  "gene_symbol": "LY6G6E",
  "gene": "UniProtKB:A0A0B4J1T7"
}